nuclear speck organization [GO:0035063] (biological process) Definition: A process that is carried out at the cellular level which results in the assembly, arrangement of constituent parts, or disassembly of nuclear specks, a class of nuclear body in which splicing factors are localized. Relationships: is a type of nuclear body organization [GO:0030575] Note: See also the cellular component term 'nuclear speck ; GO:0016607'. Sources: GOC:bf, GOC:curators Also known as: nuclear speck organisation, nuclear speckle organization, nuclear speckle assembly, nuclear speck organization and biogenesis